{
  "term_label": "DNA clamp loader activity",
  "gene_symbol": "RFC4",
  "gene_name": "Replication factor C subunit 4",
  "term_id": "GO:0003689",
  "gene": "UniProtKB:P35249"
}